{
  "term_label": "dendrite",
  "gene_symbol": "GPHN",
  "gene_name": "Gephyrin",
  "gene": "UniProtKB:Q9NQX3",
  "term_id": "GO:0030425"
}